{
  "term_id": "UNKNOWN:0001",
  "term_label": "Unknown molecular function",
  "gene_name": "Uncharacterized protein encoded by LINC02876",
  "gene_symbol": "LINC02876",
  "gene": "UniProtKB:F2Z3M2"
}